macrophage derived foam cell differentiation [GO:0010742] (biological process) Definition: The process in which a monocyte acquires the specialized features of a foam cell. A foam cell is a type of cell containing lipids in small vacuoles and typically seen in atherosclerotic lesions, as well as other conditions. Sources: GOC:add, GOC:dph, GOC:tb Relationships: is a type of foam cell differentiation [GO:0090077] Regulation: regulated by regulation of macrophage derived foam cell differentiation [GO:0010743]; RO_0002213 by positive regulation of macrophage derived foam cell differentiation [GO:0010744]; negatively regulated by negative regulation of macrophage derived foam cell differentiation [GO:0010745]